{
  "term_id": "GO:0016581",
  "gene_name": "Chromodomain-helicase-DNA-binding protein 3",
  "gene_symbol": "CHD3",
  "gene": "UniProtKB:Q12873",
  "term_label": "NuRD complex"
}